{
  "term_id": "UNKNOWN:0001",
  "gene_name": "Sperm-associated antigen 7",
  "gene_symbol": "SPAG7",
  "term_label": "Unknown molecular function",
  "gene": "UniProtKB:O75391"
}